{
  "term_label": "protein phosphatase activator activity",
  "gene_symbol": "PPP4R3C",
  "gene": "UniProtKB:Q6ZMV5",
  "gene_name": "Protein PPP4R3C",
  "term_id": "GO:0072542"
}